protein transport [GO:0015031] (biological process) Definition: The directed movement of proteins into, out of or within a cell, or between cells, by means of some agent such as a transporter or pore. Subtypes: intracellular protein transport [GO:0006886], GO:0009306, protein import [GO:0017038], endocytic hemoglobin import into cell [GO:0020028], GO:0030581, lactoferrin transport [GO:0033571], transferrin transport [GO:0033572], glycoprotein transport [GO:0034436], opsin transport [GO:0036372], GO:0042953, Golgi to plasma membrane protein transport [GO:0043001], ubiquitin-dependent endocytosis [GO:0070086], protein transport within extracellular region [GO:0071693], GO:0071806, apolipoprotein E recycling [GO:0071828], GO:0072322, microtubule-based protein transport [GO:0099118], neurotransmitter receptor transport [GO:0099637], cytosol to ERGIC protein transport [GO:0106273], protein transport to mating projection actin fusion focus [GO:1904601] Relationships: is a type of intracellular protein localization [GO:0008104]; is a type of GO:0045184; is a type of nitrogen compound transport [GO:0071705] Also known as: enzyme transport Sources: GOC:ai Regulation: positively regulated by positive regulation of protein transport [GO:0051222]; regulated by GO:0051223; negatively regulated by GO:0051224